{
  "gene_symbol": "LMBRD2",
  "gene_name": "G-protein coupled receptor-associated protein LMBRD2",
  "term_id": "UNKNOWN:0001",
  "term_label": "Unknown molecular function",
  "gene": "UniProtKB:Q68DH5"
}